{
  "gene": "UniProtKB:Q96L08",
  "term_id": "GO:0005886",
  "gene_name": "Sushi domain-containing protein 3",
  "gene_symbol": "SUSD3",
  "term_label": "plasma membrane"
}